{
  "gene": "UniProtKB:Q12891",
  "term_id": "GO:0030214",
  "gene_name": "Hyaluronidase-2",
  "term_label": "hyaluronan catabolic process",
  "gene_symbol": "HYAL2"
}